signaling [GO:0023052] (biological process) Regulation: regulated by regulation of signaling [GO:0023051]; positively regulated by positive regulation of signaling [GO:0023056]; RO_0002212 by negative regulation of signaling [GO:0023057] Relationships: is a type of regulation of biological process [GO:0050789] Also known as: biological signaling, signaling process, signalling, signalling process, single organism signaling Sources: GOC:mtg_signal, GOC:mtg_signaling_feb11, GOC:signaling Note: Note that a signal is any variable property or parameter that serves to convey information, and may be a physical entity such as a gene product or small molecule, a photon, or a change in state such as movement or voltage change. Definition: The entirety of a process in which information is transmitted within a biological system. This process begins with an active signal and ends when a cellular response has been triggered. Subtypes: cell-cell signaling [GO:0007267], motogenic signaling initiating cell movement in cerebral cortex [GO:0021807], motogenic signaling involved in postnatal olfactory bulb interneuron migration [GO:0021837], motogenic signaling involved in interneuron migration from the subpallium to the cortex [GO:0021838], extracellular matrix-cell signaling [GO:0035426]